{
  "term_id": "GO:0047555",
  "gene_name": "High affinity cAMP-specific 3',5'-cyclic phosphodiesterase 7A",
  "gene": "UniProtKB:Q13946",
  "term_label": "3',5'-cyclic-GMP phosphodiesterase activity",
  "gene_symbol": "PDE7A"
}